{
  "gene_name": "Orofacial cleft 1 candidate gene 1 protein",
  "gene_symbol": "OFCC1",
  "gene": "UniProtKB:Q8IZS5",
  "term_id": "UNKNOWN:0002",
  "term_label": "Unknown biological process"
}